negative regulation of granulocyte macrophage colony-stimulating factor production [GO:0032685] (biological process) Relationships: is a type of negative regulation of cytokine production [GO:0001818]; is a type of regulation of granulocyte macrophage colony-stimulating factor production [GO:0032645]; is a type of GO:0051248; negatively regulates granulocyte macrophage colony-stimulating factor production [GO:0032604] Also known as: down regulation of granulocyte macrophage colony-stimulating factor production, down-regulation of granulocyte macrophage colony-stimulating factor production, downregulation of granulocyte macrophage colony-stimulating factor production, negative regulation of GM-CSF production, negative regulation of granulocyte macrophage colony stimulating factor production, inhibition of granulocyte macrophage colony-stimulating factor production, negative regulation of granulocyte macrophage colony-stimulating factor biosynthetic process Definition: Any process that stops, prevents, or reduces the frequency, rate, or extent of granulocyte macrophage colony-stimulating factor production. Sources: GOC:mah